{
  "term_label": "mitochondrion",
  "term_id": "GO:0005739",
  "gene": "UniProtKB:Q14410",
  "gene_symbol": "GK2",
  "gene_name": "Glycerol kinase 2"
}